tail portion of tanycyte [GO:1990018] (cellular component) Relationships: is a type of cellular anatomical structure [GO:0110165] Definition: Elongated process of a tanycyte, devoid of cytoplasmic extensions, that courses through the hypothalamic nuclei to form small endfoot processes that terminate either on blood vessels or at the pial surface of the brain. A tanycyte is a specialized elongated ventricular ependymal cell. Sources: ISBN:0195065719, NIF_Subcellular:sao1749953771 Also known as: tail portion